{
  "gene_name": "Gamma-secretase subunit APH-1A",
  "term_label": "gamma-secretase complex",
  "gene_symbol": "APH1A",
  "gene": "UniProtKB:Q96BI3",
  "term_id": "GO:0070765"
}